regulation of somitogenesis [GO:0014807] (biological process) Definition: Any process that modulates the frequency, rate or extent of somitogenesis. Sources: GOC:mtg_muscle Relationships: is a type of regulation of anatomical structure morphogenesis [GO:0022603]; is_a regulation of multicellular organismal process [GO:0051239]; regulates somitogenesis [GO:0001756]